peptidyl-cysteine deglycation [GO:0036526] (biological process) Also known as: deglycation of N-acetylcysteine Relationships: is a type of peptidyl-cysteine modification [GO:0018198]; is a type of protein deglycation [GO:0036525] Definition: The removal of a sugar or dicarbonyl from a cysteine residue of a glycated protein. References: PMID:14568004, PMID:25416785 Sources: GOC:PARL, GOC:bf